double-strand/single-strand DNA junction binding [GO:0000406] (molecular function) Subtypes: GO:0090655 Definition: Binding to a DNA segment that contains double-stranded DNA flanked by a region of single-stranded DNA. Relationships: is a type of DNA secondary structure binding [GO:0000217] References: PMID:16781730 Sources: GOC:elh